apical dendrite arborization [GO:0150023] (BP) Definition: The process in which the anatomical structures of a dendritic tree are generated on the apical neuron side and organized into dendritic branches. References: PMID:22683681 Sources: GOC:aruk, GOC:bc Relationships: is a type of dendrite arborization [GO:0140059]; is a type of apical dendrite morphogenesis [GO:0150021]